negative regulation of leaf development [GO:1905622] (BP) Also known as: down regulation of leaf development, down-regulation of leaf development, downregulation of leaf development, inhibition of leaf development Definition: Any process that stops, prevents or reduces the frequency, rate or extent of leaf development. References: PMID:11606552 Sources: GOC:TermGenie, GO_REF:0000058 Relationships: is a type of negative regulation of developmental process [GO:0051093]; is a type of GO:0051241; is a type of regulation of leaf development [GO:2000024]; negatively regulates leaf development [GO:0048366]